{
  "term_label": "nucleus",
  "gene": "UniProtKB:P35869",
  "gene_symbol": "AHR",
  "gene_name": "Aryl hydrocarbon receptor",
  "term_id": "GO:0005634"
}